molecular adaptor activity [GO:0060090] (molecular function) Also known as: protein complex scaffold activity, protein-containing complex scaffold activity, binding, bridging Relationships: is a type of molecular_function [GO:0003674]; has part binding [GO:0005488] Subtypes: triplet codon-amino acid adaptor activity [GO:0030533], protein-macromolecule adaptor activity [GO:0030674], GO:0106260, GO:0140177 Definition: The binding activity of a molecule that brings together two or more molecules through a selective, non-covalent, often stoichiometric interaction, permitting those molecules to function in a coordinated way. Sources: GOC:mtg_MIT_16mar07, GOC:vw